negative regulation of ARF protein signal transduction [GO:0032013] (biological process) Definition: Any process that stops, prevents, or reduces the frequency, rate or extent of ARF protein signal transduction. Sources: GOC:mah Also known as: down regulation of ARF protein signal transduction, down-regulation of ARF protein signal transduction, downregulation of ARF protein signal transduction, inhibition of ARF protein signal transduction Relationships: is_a regulation of ARF protein signal transduction [GO:0032012]; is a type of negative regulation of small GTPase mediated signal transduction [GO:0051058]; negatively regulates ARF protein signal transduction [GO:0032011]